{
  "gene_name": "Interleukin-31",
  "gene": "UniProtKB:Q6EBC2",
  "term_label": "cytokine receptor binding",
  "gene_symbol": "IL31",
  "term_id": "GO:0005126"
}